C-acyltransferase activity [GO:0016408] (molecular function) Definition: Catalysis of the transfer of an acyl group to a carbon atom on the acceptor molecule. Relationships: is a type of acyltransferase activity, transferring groups other than amino-acyl groups [GO:0016747] Subtypes: acetyl-CoA C-acyltransferase activity [GO:0003988], GO:0004321, C-acetyltransferase activity [GO:0016453], C-palmitoyltransferase activity [GO:0016454], deacetylcephalosporin-C acetyltransferase activity [GO:0033813], propanoyl-CoA C-acyltransferase activity [GO:0033814], acetyl-CoA C-myristoyltransferase activity [GO:0050633] Sources: GOC:ai